{
  "term_id": "UNKNOWN:0003",
  "term_label": "Unknown cellular component",
  "gene_name": "Putative uncharacterized protein C10orf126",
  "gene": "UniProtKB:Q8N4M7",
  "gene_symbol": "C10orf126"
}